{
  "gene": "UniProtKB:Q8NGT1",
  "gene_name": "Olfactory receptor 2K2",
  "term_id": "GO:0050911",
  "gene_symbol": "OR2K2",
  "term_label": "detection of chemical stimulus involved in sensory perception of smell"
}